protein localization to cytoplasmic microtubule [GO:1905755] (biological process) Also known as: protein localisation to cytoplasmic microtubule Relationships: is a type of protein localization to microtubule [GO:0035372] References: PMID:15177031 Sources: GOC:TermGenie, GO_REF:0000087 Definition: A process in which a protein is transported to, or maintained in, a location within a cytoplasmic microtubule. Subtypes: GO:1902888, protein localization to cytoplasmic microtubule plus-end [GO:1904518]